cellobiose glucosidase activity [GO:0080079] (molecular function) Definition: Catalysis of the reaction: D-cellobiose + H2O = 2 D-glucose. Also known as: D-cellobiose glucosidase activity, cellobiose glucohydrolase activity References: PMID:15604686 Sources: RHEA:30679 Relationships: is a type of beta-glucosidase activity [GO:0008422]